{
  "gene_name": "Vesicle transport protein SEC20",
  "gene": "UniProtKB:Q12981",
  "term_label": "endoplasmic reticulum organization",
  "term_id": "GO:0007029",
  "gene_symbol": "BNIP1"
}